negative regulation of toll-like receptor 4 signaling pathway [GO:0034144] (biological process) Definition: Any process that stops, prevents, or reduces the frequency, rate, or extent of toll-like receptor 4 signaling pathway. References: PMID:16551253, PMID:17328678 Sources: GOC:add Also known as: negative regulation of TLR4 signaling pathway, negative regulation of toll-like receptor 4 signalling pathway Relationships: is a type of negative regulation of immune system process [GO:0002683]; is a type of negative regulation of signal transduction [GO:0009968]; is_a regulation of toll-like receptor 4 signaling pathway [GO:0034143]; negatively regulates toll-like receptor 4 signaling pathway [GO:0034142]